{
  "term_id": "GO:0004674",
  "gene_name": "Tau-tubulin kinase 2",
  "gene_symbol": "TTBK2",
  "term_label": "protein serine/threonine kinase activity",
  "gene": "UniProtKB:Q6IQ55"
}